{
  "term_id": "GO:0005886",
  "gene": "UniProtKB:Q9H222",
  "gene_symbol": "ABCG5",
  "term_label": "plasma membrane",
  "gene_name": "ATP-binding cassette sub-family G member 5"
}